{
  "gene_name": "Ubiquitin-conjugating enzyme E2 J2",
  "gene": "UniProtKB:Q8N2K1",
  "term_id": "GO:0005634",
  "gene_symbol": "UBE2J2",
  "term_label": "nucleus"
}